negative regulation of neutrophil mediated cytotoxicity [GO:0070954] (biological process) Subtypes: GO:0070955 Relationships: is a type of negative regulation of leukocyte mediated cytotoxicity [GO:0001911]; is a type of negative regulation of myeloid leukocyte mediated immunity [GO:0002887]; is a type of regulation of neutrophil mediated cytotoxicity [GO:0070948]; negatively regulates GO:0070942 Also known as: down regulation of neutrophil mediated cytotoxicity, down-regulation of neutrophil mediated cytotoxicity, downregulation of neutrophil mediated cytotoxicity, negative regulation of neutrophil mediated cell killing, inhibition of neutrophil mediated cytotoxicity Definition: Any process that decreases the frequency, rate or extent of the directed killing of a target cell by a neutrophil. Sources: GOC:add, GOC:mah